{
  "gene_symbol": "RAPGEF1",
  "term_id": "GO:0032486",
  "term_label": "Rap protein signal transduction",
  "gene_name": "Rap guanine nucleotide exchange factor 1",
  "gene": "UniProtKB:Q13905"
}